{
  "gene_symbol": "PADI3",
  "term_label": "cytoplasm",
  "term_id": "GO:0005737",
  "gene_name": "Protein-arginine deiminase type-3",
  "gene": "UniProtKB:Q9ULW8"
}